cytoplasmic region [GO:0099568] (cellular component) Sources: GOC:dos Definition: Any (proper) part of the cytoplasm of a single cell of sufficient size to still be considered cytoplasm. Subtypes: GO:0032838, cell cortex region [GO:0099738] Relationships: is a type of GO:0005737; is part of cytoplasm [GO:0005737]